{
  "term_id": "GO:0002502",
  "gene": "UniProtKB:O15533",
  "gene_name": "Tapasin",
  "gene_symbol": "TAPBP",
  "term_label": "peptide antigen assembly with MHC class I protein complex"
}